{
  "term_id": "GO:0005096",
  "gene_symbol": "RASAL1",
  "term_label": "GTPase activator activity",
  "gene": "UniProtKB:O95294",
  "gene_name": "RasGAP-activating-like protein 1"
}